{
  "gene_symbol": "CHD7",
  "term_label": "chromatin binding",
  "gene": "UniProtKB:Q9P2D1",
  "term_id": "GO:0003682",
  "gene_name": "Chromodomain-helicase-DNA-binding protein 7"
}